{
  "gene": "UniProtKB:P52429",
  "term_label": "glycerolipid metabolic process",
  "gene_name": "Diacylglycerol kinase epsilon",
  "gene_symbol": "DGKE",
  "term_id": "GO:0046486"
}